{
  "term_id": "UNKNOWN:0003",
  "gene_name": "Uncharacterized protein C2orf66",
  "term_label": "Unknown cellular component",
  "gene_symbol": "C2orf66",
  "gene": "UniProtKB:Q6UXQ4"
}